regulation of phenylpropanoid metabolic process [GO:2000762] (biological process) Also known as: regulation of phenylpropanoid metabolism Relationships: is_a regulation of secondary metabolic process [GO:0043455]; regulates GO:0009698 Definition: Any process that modulates the frequency, rate or extent of phenylpropanoid metabolic process. Subtypes: regulation of lignin biosynthetic process [GO:1901141], regulation of syringal lignin catabolic process [GO:1901469], GO:1903085, regulation of proanthocyanidin biosynthetic process [GO:2000029] Sources: GOC:obol